anterior lateral line development [GO:0048899] (biological process) Sources: ISBN:0125296509 Definition: The process whose specific outcome is the progression of the anterior lateral line over time, from its formation to the mature structure. The anterior lateral line consists of small sensory patches (neuromasts) located superficially on the skin or just under the skin in fluid-filled canals on the head of all fishes and most amphibians. The anterior lateral line develops from cranial ectodermal placodes situated between the eye and ear. Relationships: is a type of lateral line development [GO:0048882]; is part of anterior lateral line system development [GO:0048898] Also known as: anterior LL development